{
  "term_id": "UNKNOWN:0002",
  "gene": "UniProtKB:Q9UK58",
  "term_label": "Unknown biological process",
  "gene_name": "Cyclin-L1",
  "gene_symbol": "CCNL1"
}